{
  "gene_symbol": "SYNPO2L",
  "gene_name": "Synaptopodin 2-like protein",
  "gene": "UniProtKB:Q9H987",
  "term_id": "GO:0015629",
  "term_label": "actin cytoskeleton"
}